{
  "term_label": "regulation of transcription by RNA polymerase II",
  "gene_name": "Estrogen-related receptor gamma",
  "gene_symbol": "ESRRG",
  "term_id": "GO:0006357",
  "gene": "UniProtKB:P62508"
}